{
  "gene_symbol": "PRX",
  "gene": "UniProtKB:Q9BXM0",
  "gene_name": "Periaxin",
  "term_label": "cytoplasm",
  "term_id": "GO:0005737"
}